{
  "gene_name": "Vacuolar protein sorting-associated protein 54",
  "term_label": "syntaxin binding",
  "gene": "UniProtKB:Q9P1Q0",
  "gene_symbol": "VPS54",
  "term_id": "GO:0019905"
}